{
  "gene_symbol": "ERO1B",
  "gene": "UniProtKB:Q86YB8",
  "term_id": "GO:0015035",
  "gene_name": "ERO1-like protein beta",
  "term_label": "protein-disulfide reductase activity"
}